{
  "gene": "UniProtKB:Q86UZ6",
  "term_id": "GO:0001227",
  "gene_name": "Zinc finger and BTB domain-containing protein 46",
  "term_label": "DNA-binding transcription repressor activity, RNA polymerase II-specific",
  "gene_symbol": "ZBTB46"
}